{
  "gene_name": "Cell cycle checkpoint protein RAD1",
  "gene": "UniProtKB:O60671",
  "term_id": "UNKNOWN:0001",
  "term_label": "Unknown molecular function",
  "gene_symbol": "RAD1"
}